mitotic metaphase [GO:0000089] (BP) Note: Note that this term should not be used for direct annotation. If you are trying to make an annotation to x phase, it is likely that the correct annotation is 'regulation of x/y phase transition' or to a process which occurs during the reported phase (i.e mitotic DNA replication for mitotic S-phase). To capture the phase when a specific location or process is observed, the phase term can be used in an annotation extension (PMID:24885854) applied to a cellular component term (with the relation exists_during) or a biological process term (with the relation happens_during). Relationships: is a type of GO:0051323; is part of mitotic M phase [GO:0000087] Definition: The cell cycle phase, following prophase, during which chromosomes become aligned on the equatorial plate of the cell as part of a mitotic cell cycle. Sources: GOC:mtg_cell_cycle